{
  "gene_name": "Exosome complex component RRP46",
  "gene": "UniProtKB:Q9NQT4",
  "term_id": "GO:0034475",
  "gene_symbol": "EXOSC5",
  "term_label": "U4 snRNA 3'-end processing"
}